benzoate 4-monooxygenase activity [GO:0018664] (molecular function) Sources: EC:1.14.14.92, RHEA:18033 Definition: Catalysis of the reaction: benzoate + H+ + NADPH + O2 = 4-hydroxybenzoate + H2O + NADP+. Relationships: is a type of oxidoreductase activity, acting on paired donors, with incorporation or reduction of molecular oxygen, NAD(P)H as one donor, and incorporation of one atom of oxygen [GO:0016709] Also known as: 4-hydroxybenzoic hydroxylase activity, benzoate 4-hydroxylase activity, benzoate,NADPH:oxygen oxidoreductase (4-hydroxylating), benzoate-p-hydroxylase activity, benzoate-para-hydroxylase activity, benzoic 4-hydroxylase activity, benzoic acid 4-hydroxylase activity, p-hydroxybenzoate hydroxylase activity